negative regulation of cardiac epithelial to mesenchymal transition [GO:0062044] (biological process) Relationships: is a type of negative regulation of epithelial to mesenchymal transition [GO:0010719]; is a type of GO:0062042; negatively regulates cardiac epithelial to mesenchymal transition [GO:0060317] References: PMID:20951801 Sources: GOC:BFH, GOC:rph Subtypes: negative regulation of endocardial cushion to mesenchymal transition [GO:0140050], negative regulation of epithelial to mesenchymal transition involved in endocardial cushion formation [GO:1905006] Definition: Any process that stops or decreases the rate, frequency or extent of cardiac epithelial to mesenchymal transition, a transition where a cardiac epithelial cell loses apical/basolateral polarity, severs intercellular adhesive junctions, degrades basement membrane components and becomes a migratory mesenchymal cell.